early endosome to recycling endosome transport [GO:0061502] (biological process) Definition: The directed movement of substances, in membrane-bounded vesicles, from the early sorting endosomes to the recycling endosomes. Relationships: is a type of GO:0098927; occurs in cytoplasm [GO:0005737] References: PMID:21474295 Sources: GOC:dph, GOC:kmv Regulation: regulated by regulation of early endosome to recycling endosome transport [GO:1902954]; positively regulated by GO:1902955